{
  "gene_name": "Putative protein MSS51 homolog, mitochondrial",
  "gene": "UniProtKB:Q4VC12",
  "term_id": "UNKNOWN:0002",
  "gene_symbol": "MSS51",
  "term_label": "Unknown biological process"
}